{
  "gene": "UniProtKB:Q8TAY7",
  "gene_symbol": "FAM110D",
  "term_label": "Unknown biological process",
  "term_id": "UNKNOWN:0002",
  "gene_name": "Protein FAM110D"
}